{
  "gene": "UniProtKB:P35914",
  "term_id": "GO:0046951",
  "gene_name": "Hydroxymethylglutaryl-CoA lyase, mitochondrial",
  "gene_symbol": "HMGCL",
  "term_label": "ketone body biosynthetic process"
}